{
  "gene_symbol": "FCGR2A",
  "gene": "UniProtKB:P12318",
  "term_label": "antibody-dependent cellular cytotoxicity",
  "term_id": "GO:0001788",
  "gene_name": "Low affinity immunoglobulin gamma Fc region receptor II-a"
}